{
  "term_id": "GO:0003723",
  "gene_name": "GTP-binding protein 4",
  "gene": "UniProtKB:Q9BZE4",
  "term_label": "RNA binding",
  "gene_symbol": "GTPBP4"
}